{
  "gene_name": "Small nuclear ribonucleoprotein G",
  "gene": "UniProtKB:P62308",
  "term_id": "GO:0000398",
  "term_label": "mRNA splicing, via spliceosome",
  "gene_symbol": "SNRPG"
}